{
  "gene_symbol": "ADAT3",
  "gene": "UniProtKB:Q96EY9",
  "term_label": "Unknown molecular function",
  "gene_name": "Probable inactive tRNA-specific adenosine deaminase-like protein 3",
  "term_id": "UNKNOWN:0001"
}